{
  "gene_name": "Phospholipid phosphatase-related protein type 2",
  "gene": "UniProtKB:Q96GM1",
  "term_label": "phospholipid metabolic process",
  "term_id": "GO:0006644",
  "gene_symbol": "PLPPR2"
}